parallel actin filament bundle assembly [GO:0030046] (biological process) Relationships: is a type of actin filament bundle assembly [GO:0051017] Definition: Assembly of actin filament bundles in which the filaments are tightly packed (approximately 10-20 nm apart) and oriented with the same polarity. Subtypes: microvillar actin bundle assembly [GO:0030034], formin-nucleated actin cable assembly [GO:0070649] Sources: GOC:mah, ISBN:0815316194